{
  "term_label": "cytoplasmic vesicle",
  "term_id": "GO:0031410",
  "gene": "UniProtKB:Q658Y4",
  "gene_name": "Protein FAM91A1",
  "gene_symbol": "FAM91A1"
}